{
  "term_id": "UNKNOWN:0002",
  "gene_symbol": "ABO",
  "term_label": "Unknown biological process",
  "gene_name": "Histo-blood group ABO system transferase",
  "gene": "UniProtKB:P16442"
}